regulation of carbohydrate metabolic process [GO:0006109] (biological process) Relationships: is a type of regulation of primary metabolic process [GO:0080090]; RO_0002211 carbohydrate metabolic process [GO:0005975] Also known as: regulation of carbohydrate metabolism Definition: Any process that modulates the frequency, rate or extent of the chemical reactions and pathways involving carbohydrates. Sources: GOC:go_curators Subtypes: regulation of isopentenyl diphosphate biosynthetic process, methylerythritol 4-phosphate pathway [GO:0010322], regulation of glucose metabolic process [GO:0010906], regulation of polysaccharide metabolic process [GO:0032881], regulation of carbohydrate biosynthetic process [GO:0043255], GO:0043470, GO:0045912, positive regulation of carbohydrate metabolic process [GO:0045913], regulation of raffinose metabolic process [GO:0080091], regulation of trehalose metabolic process [GO:0090062], regulation of glyoxylate cycle [GO:2000874]